{
  "term_label": "Unknown biological process",
  "gene": "UniProtKB:Q8NHB7",
  "gene_name": "Olfactory receptor 5K1",
  "gene_symbol": "OR5K1",
  "term_id": "UNKNOWN:0002"
}